{
  "gene_symbol": "C12orf54",
  "gene": "UniProtKB:Q6X4T0",
  "term_label": "Unknown molecular function",
  "gene_name": "Uncharacterized protein C12orf54",
  "term_id": "UNKNOWN:0001"
}